{
  "gene_name": "Cdc42 effector protein 2",
  "term_label": "small GTPase binding",
  "gene_symbol": "CDC42EP2",
  "term_id": "GO:0031267",
  "gene": "UniProtKB:O14613"
}